{
  "gene_symbol": "PMP2",
  "term_label": "fatty acid binding",
  "gene": "UniProtKB:P02689",
  "gene_name": "Myelin P2 protein",
  "term_id": "GO:0005504"
}